{
  "gene": "UniProtKB:Q15058",
  "term_id": "GO:0005874",
  "gene_symbol": "KIF14",
  "gene_name": "Kinesin-like protein KIF14",
  "term_label": "microtubule"
}